{
  "gene": "UniProtKB:Q5VZE5",
  "gene_symbol": "NAA35",
  "gene_name": "N-alpha-acetyltransferase 35, NatC auxiliary subunit",
  "term_label": "Unknown molecular function",
  "term_id": "UNKNOWN:0001"
}